mycotoxin metabolic process [GO:0043385] (biological process) Definition: The chemical reactions and pathways involving a mycotoxin, any poisonous substance produced by a fungus. Sources: GOC:jl Also known as: mycotoxin metabolism Relationships: is a type of toxin metabolic process [GO:0009404] Subtypes: mycotoxin biosynthetic process [GO:0043386], mycotoxin catabolic process [GO:0043387], aflatoxin metabolic process [GO:0046222]